{
  "gene_name": "Histone-lysine N-methyltransferase EZH1",
  "term_label": "histone H3K27 methyltransferase activity",
  "gene": "UniProtKB:Q92800",
  "term_id": "GO:0046976",
  "gene_symbol": "EZH1"
}